{
  "gene": "UniProtKB:Q96GX5",
  "term_label": "regulation of mitotic cell cycle",
  "term_id": "GO:0007346",
  "gene_name": "Serine_threonine-protein kinase greatwall",
  "gene_symbol": "MASTL"
}